geranylgeranyltransferase-III complex [GO:0170069] (cellular component) Definition: A protein-containing complex that catalyzes the transfer of a geranyl-geranyl group from geranylgeranyl pyrophosphate to a mono-farnsylated substrate. In humans, the complex is comprised of a prenyltransferase alpha subunit, PTAR1 and beta subunit, RabGGTB, while in budding yeast the prenyltransferase complex contains Ecm9p, the alpha subunit and Bet2p, the beta subunit. References: PMID:32128853, PMID:33035318, PMID:35628237, PMID:40049413 Also known as: GGT3, GGTase-3 complex, GGTase-III complex, GGTase3 complex, geranylgeranyltransferase type 3 complex, geranylgeranyltransferase type-3 complex, type-III geranylgeranyltransferase complex Relationships: is a type of transferase complex [GO:1990234]; is part of cytosol [GO:0005829]